positive regulation of endocytic recycling [GO:2001137] (biological process) Definition: Any process that activates or increases the frequency, rate or extent of endocytic recycling. Also known as: positive regulation of retrograde transport of endocytic vesicles Relationships: is a type of positive regulation of intracellular transport [GO:0032388]; is a type of regulation of endocytic recycling [GO:2001135]; positively regulates endocytic recycling [GO:0032456] Sources: GOC:obol Subtypes: positive regulation of endosome to plasma membrane protein transport [GO:1905751]